box C/D methylation guide snoRNP complex [GO:0031428] (cellular component) References: PMID:11842104, PMID:17284456 Sources: ISBN:0879695897 Definition: A ribonucleoprotein complex containing a box C/D type RNA that is capable of ribose-2'-O-methylation of target RNAs. Box C/D type RNAs are widespread in eukaryotes and in Archaea, suggesting that an RNA-based guide mechanism for directing specific RNA 2'-O-ribose methylations was present in the common ancestor of Archaea and Eukarya. Also known as: box C/D snoRNP ribose 2'-O methylase complex, box C/D sRNP complex, box C/D small nucleolar ribonucleoprotein complex, box C/D snoRNP complex, box C/D snoRNP ribose-2'-O-methyltransferase complex Relationships: is a type of box C/D RNP complex [GO:0170049]